regulation of anthocyanin metabolic process [GO:0031537] (biological process) Definition: Any process that modulates the frequency, rate or extent of chemical reactions and pathways involving anthocyanins. Sources: GOC:mah Also known as: regulation of anthocyanin metabolism Subtypes: negative regulation of anthocyanin metabolic process [GO:0031538], positive regulation of anthocyanin metabolic process [GO:0031539], regulation of anthocyanin biosynthetic process [GO:0031540], regulation of anthocyanin catabolic process [GO:1900000] Relationships: is a type of GO:0080090; regulates GO:0046283